adult chitin-based cuticle development [GO:0008365] (biological process) Definition: Synthesis and deposition of the chitin-based cuticle of adults following the apolysis of the pupal cuticle. The adult insect cuticle contains cuticullin, a protein epicuticle and a lamellate procuticle. An example of this process is adult chitin-based cuticle development in Drosophila melanogaster. Relationships: is a type of chitin-based cuticle development [GO:0040003] Sources: GOC:bf, GOC:mtg_sensu, ISBN:0879694238 Also known as: adult cuticle anabolism, adult cuticle biosynthetic process, adult cuticle formation, adult cuticle synthesis, adult chitin-based cuticle anabolism, adult chitin-based cuticle biosynthetic process, adult chitin-based cuticle formation, adult chitin-based cuticle synthesis